monodictyphenone catabolic process [GO:1900814] (biological process) Also known as: monodictyphenone breakdown, monodictyphenone catabolism, monodictyphenone degradation Sources: GOC:TermGenie, GOC:di Relationships: is a type of phenol-containing compound catabolic process [GO:0019336]; is a type of ketone catabolic process [GO:0042182]; is a type of carboxylic acid catabolic process [GO:0046395]; is a type of secondary metabolite catabolic process [GO:0090487]; is a type of monodictyphenone metabolic process [GO:1900813] Definition: The chemical reactions and pathways resulting in the breakdown of monodictyphenone.